{
  "gene_symbol": "EPS15",
  "gene_name": "Epidermal growth factor receptor substrate 15",
  "term_id": "GO:0016197",
  "term_label": "endosomal transport",
  "gene": "UniProtKB:P42566"
}